{
  "gene": "UniProtKB:P98170",
  "term_id": "GO:0090263",
  "term_label": "positive regulation of canonical Wnt signaling pathway",
  "gene_name": "E3 ubiquitin-protein ligase XIAP",
  "gene_symbol": "XIAP"
}